B800-820 antenna complex [GO:0030081] (cellular component) Also known as: LH3 complex, light harvesting complex III Relationships: is_a GO:0032991; is part of light-harvesting complex, peripheral complex [GO:0030079] Definition: Protein-pigment complex that absorbs light at 800 and 820 nm; is peripherally associated to the bacterial reaction center; transfers excitation energy to the B875 antenna complex. Sources: GOC:kd, GOC:lr